{
  "gene_name": "Sphingolipid delta(4)-desaturase DES1",
  "gene_symbol": "DEGS1",
  "term_label": "sphingolipid delta-4 desaturase activity",
  "gene": "UniProtKB:O15121",
  "term_id": "GO:0042284"
}